{
  "term_label": "negative regulation of TOR signaling",
  "gene": "UniProtKB:Q70Z35",
  "term_id": "GO:0032007",
  "gene_name": "Phosphatidylinositol 3,4,5-trisphosphate-dependent Rac exchanger 2 protein",
  "gene_symbol": "PREX2"
}